aralkylamine N-acetyltransferase activity [GO:0004059] (molecular function) Definition: Catalysis of the reaction: acetyl-CoA + an aralkylamine = CoA + an N-acetylaralkylamine. Sources: EC:2.3.1.87 Also known as: serotonin N-acetyltransferase activity, serotonin acetylase activity, serotonin acetyltransferase activity, AANAT activity, acetyl-CoA:2-arylethylamine N-acetyltransferase activity, arylalkylamine N-acetyltransferase activity, melatonin rhythm enzyme activity Relationships: is a type of N-acetyltransferase activity [GO:0008080]